{
  "term_id": "GO:0045121",
  "term_label": "membrane raft",
  "gene_name": "T-cell surface glycoprotein CD4",
  "gene_symbol": "CD4",
  "gene": "UniProtKB:P01730"
}